{
  "gene_symbol": "MGST1",
  "gene": "UniProtKB:P10620",
  "gene_name": "Microsomal glutathione S-transferase 1",
  "term_label": "Unknown biological process",
  "term_id": "UNKNOWN:0002"
}